{
  "gene_symbol": "MAPK9",
  "gene_name": "Mitogen-activated protein kinase 9",
  "term_id": "GO:0005737",
  "gene": "UniProtKB:P45984",
  "term_label": "cytoplasm"
}